{
  "gene": "UniProtKB:Q9Y657",
  "term_label": "Unknown molecular function",
  "term_id": "UNKNOWN:0001",
  "gene_name": "Spindlin-1",
  "gene_symbol": "SPIN1"
}